{
  "term_id": "GO:0030215",
  "gene_symbol": "SEMA3A",
  "gene_name": "Semaphorin-3A",
  "gene": "UniProtKB:Q14563",
  "term_label": "semaphorin receptor binding"
}